{
  "gene": "UniProtKB:P0C7L1",
  "gene_symbol": "SPINK8",
  "term_id": "UNKNOWN:0003",
  "term_label": "Unknown cellular component",
  "gene_name": "Serine protease inhibitor Kazal-type 8"
}